alpha-zeacarotene biosynthetic process [GO:1901821] (biological process) References: PMID:6060456 Sources: GOC:TermGenie, GOC:yaf, UniPathway:UPA00804 Also known as: alpha-zeacarotene anabolism, alpha-zeacarotene biosynthesis, alpha-zeacarotene formation, alpha-zeacarotene synthesis Relationships: is a type of GO:0016117; is a type of carotene biosynthetic process [GO:0016120] Definition: The chemical reactions and pathways resulting in the formation of alpha-zeacarotene.